positive regulation of peptide secretion [GO:0002793] (biological process) Sources: GOC:add Definition: Any process that activates or increases the frequency, rate, or extent of peptide secretion. Also known as: up regulation of peptide secretion, up-regulation of peptide secretion, upregulation of peptide secretion, activation of peptide secretion, stimulation of peptide secretion Relationships: is a type of regulation of peptide secretion [GO:0002791]; is a type of positive regulation of secretion [GO:0051047]; positively regulates GO:0002790 Subtypes: GO:0002796, positive regulation of peptide hormone secretion [GO:0090277]